{
  "term_id": "UNKNOWN:0003",
  "gene_symbol": "PNMA2",
  "gene": "UniProtKB:Q9UL42",
  "term_label": "Unknown cellular component",
  "gene_name": "Paraneoplastic antigen Ma2"
}